positive regulation of conidiophore stalk development [GO:0070801] (biological process) Sources: GOC:mah Definition: Any process that activates or increases the frequency, rate or extent of conidiophore stalk development, a process that leads to the formation of a conidiophore stalk. The conidiophore stalk is part of a specialized hypha that extends aerially from the growth substrate and supports structures from which conidia, or asexual spores, develop. Relationships: is_a GO:0070795; is a type of regulation of conidiophore stalk development [GO:0070799]; positively regulates conidiophore stalk development [GO:0070788]